dAMP binding [GO:0032562] (MF) Relationships: is a type of GO:0032558; is a type of anion binding [GO:0043168] Sources: GOC:mah Definition: Binding to dAMP, deoxyadenosine monophosphate.